{
  "gene_name": "TNF receptor-associated factor 2",
  "term_id": "GO:0004842",
  "gene_symbol": "TRAF2",
  "term_label": "ubiquitin-protein transferase activity",
  "gene": "UniProtKB:Q12933"
}